sulfur amino acid transmembrane transporter activity [GO:0000099] (molecular function) Sources: GOC:ai, GOC:mtg_transport, ISBN:0815340729 Also known as: sulfur amino acid transporter activity, sulphur amino acid transporter activity, sulphur amino acid transmembrane transporter activity Definition: Enables the transfer of sulfur amino acids from one side of a membrane to the other. Sulphur amino acids contain sulfur in the form of cystine, methionine or their derivatives. Subtypes: 3-sulfino-L-alanine: proton, glutamate antiporter activity [GO:0000514], L-cystine transmembrane transporter activity [GO:0015184], cystine:glutamate antiporter activity [GO:0015327], cysteine transmembrane transporter activity [GO:0033229], GO:0043865 Relationships: is a type of carboxylic acid transmembrane transporter activity [GO:0046943]; is a type of sulfur compound transmembrane transporter activity [GO:1901682]